{
  "gene": "UniProtKB:P0C854",
  "term_label": "Unknown cellular component",
  "term_id": "UNKNOWN:0003",
  "gene_name": "Putative cat eye syndrome critical region protein 9",
  "gene_symbol": "CECR9"
}